{
  "term_label": "negative regulation of TOR signaling",
  "gene_symbol": "DDIT4",
  "gene_name": "DNA damage-inducible transcript 4 protein",
  "term_id": "GO:0032007",
  "gene": "UniProtKB:Q9NX09"
}